N,N-dimethylformamidase activity [GO:0050116] (molecular function) Relationships: is a type of hydrolase activity, acting on carbon-nitrogen (but not peptide) bonds, in linear amides [GO:0016811] Also known as: DMFase activity, N,N-dimethylformamide amidohydrolase activity, dimethylformamidase activity Sources: EC:3.5.1.56, RHEA:19517 Definition: Catalysis of the reaction: N,N-dimethylformamide + H2O = dimethylamine + formate.